cobinamide phosphate guanylyltransferase activity [GO:0008820] (molecular function) Sources: RHEA:22712 Also known as: AdoCbi kinase/AdoCbi-phosphate guanylyltransferase, adenosylcobinamide kinase/adenosylcobinamide-phosphate guanylyltransferase, GTP:adenosylcobinamide-phosphate guanylyltransferase activity, GTP:cobinamide phosphate guanylyltransferase activity, adenosylcobinamide-phosphate guanylyltransferase activity, CobU Definition: Catalysis of the reaction: adenosylcobinamide phosphate + GTP + 2 H+ = adenosylcobinamide-GDP + diphosphate. Relationships: is a type of guanylyltransferase activity [GO:0070568]